{
  "gene_symbol": "STON1",
  "gene": "UniProtKB:Q9Y6Q2",
  "gene_name": "Stonin-1",
  "term_id": "GO:0030100",
  "term_label": "regulation of endocytosis"
}